pigment accumulation in response to UV light [GO:0043478] (biological process) Subtypes: pigment accumulation in tissues in response to UV light [GO:0043479] Relationships: is a type of response to UV [GO:0009411]; is a type of pigment accumulation [GO:0043476] Sources: GOC:jl Definition: The aggregation of coloring matter in a particular location in an organism, tissue or cell, occurring in response to a UV light stimulus.